pentaerythritol tetranitrate metabolic process [GO:0018954] (biological process) Sources: UM-BBD_pathwayID:petn Relationships: is a type of xenobiotic metabolic process [GO:0006805] Also known as: pentaerythritol tetranitrate metabolism Definition: The chemical reactions and pathways involving pentaerythritol tetranitrate, C(CH2-O-NO2)4, a substance produced for use as an explosive and a vasodilator.